{
  "gene": "UniProtKB:O75385",
  "term_id": "GO:0042594",
  "gene_symbol": "ULK1",
  "term_label": "response to starvation",
  "gene_name": "Serine_threonine-protein kinase ULK1"
}